trans-2-enoyl-CoA reductase (NADH) activity [GO:0050343] (molecular function) Definition: Catalysis of the reaction: acyl-CoA + NAD+ = trans-didehydroacyl-CoA + NADH. Also known as: acyl-CoA:NAD+ trans-2-oxidoreductase activity Relationships: is a type of oxidoreductase activity, acting on the CH-CH group of donors, NAD or NADP as acceptor [GO:0016628] Sources: EC:1.3.1.44